{
  "gene_symbol": "HYCC2",
  "gene": "UniProtKB:Q8IXS8",
  "term_label": "Unknown molecular function",
  "gene_name": "Hyccin 2",
  "term_id": "UNKNOWN:0001"
}